positive regulation of vasculature development [GO:1904018] (biological process) Subtypes: positive regulation of angiogenesis [GO:0045766] Definition: Any process that activates or increases the frequency, rate or extent of vasculature development. Also known as: up regulation of vasculature development, up-regulation of vasculature development, upregulation of vasculature development, activation of vasculature development, activation of vascular system development, positive regulation of vascular system development, up regulation of vascular system development, up-regulation of vascular system development, upregulation of vascular system development Relationships: is a type of positive regulation of developmental process [GO:0051094]; is a type of positive regulation of multicellular organismal process [GO:0051240]; is a type of regulation of vasculature development [GO:1901342]; positively regulates vasculature development [GO:0001944] References: PMID:21472453 Sources: GOC:TermGenie, GO_REF:0000058